{
  "gene_name": "Zinc finger SWIM domain-containing protein 3",
  "gene": "UniProtKB:Q96MP5",
  "term_id": "UNKNOWN:0002",
  "term_label": "Unknown biological process",
  "gene_symbol": "ZSWIM3"
}